{
  "gene_symbol": "CPLX3",
  "term_label": "synaptic vesicle exocytosis",
  "term_id": "GO:0016079",
  "gene": "UniProtKB:Q8WVH0",
  "gene_name": "Complexin-3"
}